complement component C3dg receptor activity [GO:0001859] (molecular function) Relationships: is a type of complement receptor activity [GO:0004875]; has part complement component C3dg binding [GO:0001853] Sources: GOC:add, GOC:signaling, ISBN:0781735149 Definition: Combining with the C3dg product of the complement cascade and transmitting the signal from one side of the membrane to the other to initiate a change in cell activity.